{
  "term_label": "lipid oxidation",
  "gene": "UniProtKB:P16050",
  "term_id": "GO:0034440",
  "gene_name": "Polyunsaturated fatty acid lipoxygenase ALOX15",
  "gene_symbol": "ALOX15"
}